{
  "term_label": "Unknown cellular component",
  "term_id": "UNKNOWN:0003",
  "gene": "UniProtKB:Q8N7X8",
  "gene_name": "SIGLEC family-like protein 1",
  "gene_symbol": "SIGLECL1"
}